{
  "term_id": "GO:0003823",
  "gene_name": "Ig-like domain-containing protein (Fragment)",
  "term_label": "antigen binding",
  "gene": "UniProtKB:A0A0J9YY99",
  "gene_symbol": "A0A0J9YY99"
}